{
  "term_label": "SCF-dependent proteasomal ubiquitin-dependent protein catabolic process",
  "gene": "UniProtKB:Q8NI29",
  "gene_symbol": "FBXO27",
  "gene_name": "F-box only protein 27",
  "term_id": "GO:0031146"
}